{
  "gene_symbol": "NDUFAF3",
  "gene": "UniProtKB:Q9BU61",
  "term_id": "GO:0032981",
  "gene_name": "NADH dehydrogenase [ubiquinone] 1 alpha subcomplex assembly factor 3",
  "term_label": "mitochondrial respiratory chain complex I assembly"
}